trans-permethrin hydrolase activity [GO:0102209] (molecular function) Definition: Catalysis of the reaction: (-)-trans-permethrin + H2O = H+ + (3-phenoxyphenyl)methanol + (1S,3R)-3-(2,2-dichlorovinyl)-2,2-dimethylcyclopropanecarboxylate. Sources: EC:3.1.1.88, GOC:pz Relationships: is a type of GO:0052689